{
  "term_id": "UNKNOWN:0002",
  "gene_symbol": "MEDAG",
  "gene": "UniProtKB:Q5VYS4",
  "gene_name": "Mesenteric estrogen-dependent adipogenesis protein",
  "term_label": "Unknown biological process"
}